{
  "term_id": "GO:0016485",
  "gene_name": "Cysteine protease ATG4B",
  "gene": "UniProtKB:Q9Y4P1",
  "gene_symbol": "ATG4B",
  "term_label": "protein processing"
}